{
  "term_id": "GO:0008104",
  "gene_symbol": "SEPTIN11",
  "gene_name": "Septin-11",
  "gene": "UniProtKB:Q9NVA2",
  "term_label": "intracellular protein localization"
}